{
  "gene_name": "Myeloid-associated differentiation marker",
  "gene": "UniProtKB:Q96S97",
  "gene_symbol": "MYADM",
  "term_id": "GO:0005911",
  "term_label": "cell-cell junction"
}